{
  "term_id": "GO:0090575",
  "gene": "UniProtKB:P19793",
  "gene_symbol": "RXRA",
  "gene_name": "Retinoic acid receptor RXR-alpha",
  "term_label": "RNA polymerase II transcription regulator complex"
}